{
  "term_label": "Unknown molecular function",
  "gene_symbol": "NPIPA7",
  "gene": "UniProtKB:E9PJI5",
  "gene_name": "Nuclear pore complex-interacting protein family member A7",
  "term_id": "UNKNOWN:0001"
}